{
  "term_label": "membrane",
  "gene_symbol": "TAS2R16",
  "gene": "UniProtKB:Q9NYV7",
  "gene_name": "Taste receptor type 2 member 16",
  "term_id": "GO:0016020"
}